sex chromosome [GO:0000803] (cellular component) Definition: A chromosome involved in sex determination. Sources: GOC:elh Subtypes: W chromosome [GO:0000804], X chromosome [GO:0000805], Y chromosome [GO:0000806], Z chromosome [GO:0000807], XY body [GO:0001741], GO:0098577, GO:0098579 Relationships: is a type of chromosome [GO:0005694]